premeiotic DNA replication [GO:0006279] (biological process) Sources: GOC:TermGenie, GOC:ai, GO_REF:0000060 Definition: The replication of DNA that precedes meiotic cell division. Relationships: is a type of nuclear DNA replication [GO:0033260]; is a type of GO:1903046 Also known as: DNA replication involved in S phase involved in meiotic cell cycle, DNA replication involved in S-phase involved in meiotic cell cycle, meiotic cell cycle DNA replication, meiotic nuclear cell cycle DNA replication, nuclear cell cycle DNA replication involved in meiotic cell cycle, DNA replication during S phase involved in meiotic cell cycle, meiotic DNA replication, meiotic DNA synthesis, premeiotic DNA synthesis